regulation of pericentric heterochromatin formation [GO:0090052] (biological process) Definition: Any process that modulates the frequency, rate or extent of heterochromatin formation at the centromere. Chromatin silencing at the centromere is the repression of transcription of centromeric DNA by altering the structure of chromatin. Relationships: is a type of GO:0031445; RO_0002211 GO:0031508 Sources: GOC:dph, GOC:tb Subtypes: positive regulation of pericentric heterochromatin formation [GO:0090053] Also known as: regulation of chromatin silencing at centromere, regulation of pericentric heterochromatin assembly